{
  "gene": "UniProtKB:O15503",
  "gene_name": "Insulin-induced gene 1 protein",
  "term_id": "GO:0032937",
  "gene_symbol": "INSIG1",
  "term_label": "SREBP-SCAP-Insig complex"
}